negative regulation of apoptotic signaling pathway [GO:2001234] (biological process) Definition: Any process that stops, prevents or reduces the frequency, rate or extent of apoptotic signaling pathway. Sources: GOC:mtg_apoptosis Also known as: negative regulation of apoptotic signalling pathway Relationships: is a type of negative regulation of signal transduction [GO:0009968]; is a type of negative regulation of apoptotic process [GO:0043066]; is a type of GO:2001233; negatively regulates apoptotic signaling pathway [GO:0097190] Subtypes: negative regulation of release of cytochrome c from mitochondria [GO:0090201], GO:1901029, negative regulation of apoptosome assembly [GO:1905101], negative regulation of extrinsic apoptotic signaling pathway [GO:2001237], negative regulation of intrinsic apoptotic signaling pathway [GO:2001243]